{
  "term_label": "regulation of transcription by RNA polymerase II",
  "gene_name": "Forkhead box protein D3",
  "gene_symbol": "FOXD3",
  "term_id": "GO:0006357",
  "gene": "UniProtKB:Q9UJU5"
}